{
  "gene": "UniProtKB:Q9Y5X4",
  "term_id": "UNKNOWN:0003",
  "term_label": "Unknown cellular component",
  "gene_name": "Photoreceptor-specific nuclear receptor",
  "gene_symbol": "NR2E3"
}